histone H3K9me2 methyltransferase activity [GO:0140947] (molecular function) Sources: RHEA:60288 Relationships: is a type of histone H3K9 methyltransferase activity [GO:0046974] Also known as: histone H3-K9 trimethylation, histone H3K9 trimethylation, histone H3K9me2 methylase activity, histone dimethyl-lysine(H3K9) N-methyltransferase activity (H3-K9 specific) Definition: Catalysis of the reaction: N6,N6-dimethyl-L-lysyl9-[histone H3] + S-adenosyl-L-methionine = H+ + N6,N6,N6-trimethyl-L-lysyl9-[histone H3] + S-adenosyl-L-homocysteine. This reaction is the addition of a single methyl group to the dimethylated lysine residue at position 9 of histone H3, producing histone H3K9me3. Note: Comment: Note that the residue position corresponds to the canonical human H3 histone (UniProtKB:P84243); this residue is conserved across all eukaryotes. Residue 1 is the first residue following removal of the initiating Methionine (Met). Note that each histone is encoded by multiple genes, and sequences may vary across different genes within an organism.